{
  "term_label": "Unknown cellular component",
  "gene_name": "Mitoguardin 1",
  "gene": "UniProtKB:Q8NAN2",
  "gene_symbol": "MIGA1",
  "term_id": "UNKNOWN:0003"
}